{
  "term_id": "GO:0005886",
  "gene_name": "Multiple PDZ domain protein",
  "gene_symbol": "MPDZ",
  "gene": "UniProtKB:O75970",
  "term_label": "plasma membrane"
}